{
  "term_label": "cytosol",
  "gene_name": "Proteasome subunit beta type-5",
  "gene": "UniProtKB:P28074",
  "gene_symbol": "PSMB5",
  "term_id": "GO:0005829"
}